{
  "gene": "UniProtKB:Q6ZS92",
  "gene_symbol": "Q6ZS92",
  "term_label": "Unknown biological process",
  "gene_name": "Putative uncharacterized protein FLJ45721",
  "term_id": "UNKNOWN:0002"
}